{
  "gene_symbol": "TNNT2",
  "gene_name": "Troponin T, cardiac muscle",
  "gene": "UniProtKB:P45379",
  "term_label": "cardiac muscle contraction",
  "term_id": "GO:0060048"
}